{
  "gene_name": "Carboxypeptidase D",
  "term_id": "GO:0006518",
  "term_label": "peptide metabolic process",
  "gene": "UniProtKB:O75976",
  "gene_symbol": "CPD"
}